{
  "gene_symbol": "INS-IGF2",
  "term_id": "UNKNOWN:0002",
  "term_label": "Unknown biological process",
  "gene": "UniProtKB:F8WCM5",
  "gene_name": "Insulin, isoform 2"
}